{
  "gene_symbol": "KLB",
  "gene_name": "Beta-klotho",
  "term_label": "Unknown molecular function",
  "gene": "UniProtKB:Q86Z14",
  "term_id": "UNKNOWN:0001"
}